{
  "gene_name": "Cyclic nucleotide-gated cation channel beta-1",
  "term_id": "GO:0030553",
  "gene_symbol": "CNGB1",
  "gene": "UniProtKB:Q14028",
  "term_label": "cGMP binding"
}